{
  "term_id": "GO:0009897",
  "gene": "UniProtKB:Q8NI17",
  "gene_symbol": "IL31RA",
  "gene_name": "Interleukin-31 receptor subunit alpha",
  "term_label": "external side of plasma membrane"
}